{
  "gene": "UniProtKB:P12883",
  "term_id": "GO:0060048",
  "term_label": "cardiac muscle contraction",
  "gene_symbol": "MYH7",
  "gene_name": "Myosin-7"
}